{
  "gene_name": "Calcitonin receptor",
  "gene_symbol": "CALCR",
  "term_label": "calcitonin receptor activity",
  "gene": "UniProtKB:P30988",
  "term_id": "GO:0004948"
}